{
  "gene": "UniProtKB:Q9BXW6",
  "term_label": "plasma membrane",
  "gene_symbol": "OSBPL1A",
  "term_id": "GO:0005886",
  "gene_name": "Oxysterol-binding protein-related protein 1"
}